maintenance of mitochondrion location [GO:0051659] (biological process) Sources: GOC:ai, GOC:dph, GOC:tb Definition: Any process in which a mitochondrion is maintained in a specific location within a cell and prevented from moving elsewhere. Relationships: is a type of mitochondrion localization [GO:0051646]; is a type of maintenance of organelle location [GO:0051657] Also known as: maintenance of mitochondria localization, maintenance of mitochondrion localization